cellular response to methanol [GO:0071405] (biological process) Relationships: is a type of GO:0033986; is a type of GO:0097306 Definition: Any process that results in a change in state or activity of a cell (in terms of movement, secretion, enzyme production, gene expression, etc.) as a result of a methanol stimulus. Sources: GOC:mah